{
  "term_id": "GO:0038203",
  "gene": "UniProtKB:P85299",
  "gene_symbol": "PRR5",
  "gene_name": "Proline-rich protein 5",
  "term_label": "TORC2 signaling"
}